{
  "gene_name": "Oxidative stress-induced growth inhibitor 1",
  "gene": "UniProtKB:Q9UJX0",
  "gene_symbol": "OSGIN1",
  "term_label": "growth factor activity",
  "term_id": "GO:0008083"
}